{
  "gene_name": "Ropporin-1A",
  "gene_symbol": "ROPN1",
  "term_id": "GO:0030317",
  "term_label": "flagellated sperm motility",
  "gene": "UniProtKB:Q9HAT0"
}